{
  "gene_name": "Outer dense fiber protein 3-like protein 2",
  "term_id": "GO:0005881",
  "gene": "UniProtKB:Q3SX64",
  "gene_symbol": "ODF3L2",
  "term_label": "cytoplasmic microtubule"
}